{
  "gene": "UniProtKB:O14977",
  "term_label": "positive regulation of polyamine transmembrane transport",
  "gene_symbol": "AZIN1",
  "term_id": "GO:1902269",
  "gene_name": "Antizyme inhibitor 1"
}